{
  "gene_symbol": "ERVK13-1",
  "gene_name": "Endogenous retrovirus group K member 13-1 Env polyprotein",
  "term_label": "Unknown molecular function",
  "gene": "UniProtKB:Q9NX77",
  "term_id": "UNKNOWN:0001"
}